negative regulation of mechanosensory behavior [GO:1905791] (biological process) References: PMID:8692859 Sources: GOC:TermGenie, GO_REF:0000058 Relationships: is a type of negative regulation of response to external stimulus [GO:0032102]; is a type of negative regulation of behavior [GO:0048521]; is a type of regulation of mechanosensory behavior [GO:1905790]; negatively regulates mechanosensory behavior [GO:0007638] Also known as: down regulation of behavioral response to mechanical stimulus, down regulation of behavioural response to mechanical stimulus, down regulation of mechanosensory behavior, down regulation of mechanosensory behaviour, down-regulation of behavioral response to mechanical stimulus, down-regulation of behavioural response to mechanical stimulus, down-regulation of mechanosensory behavior, down-regulation of mechanosensory behaviour, downregulation of behavioral response to mechanical stimulus, downregulation of behavioural response to mechanical stimulus, downregulation of mechanosensory behavior, downregulation of mechanosensory behaviour, negative regulation of behavioral response to mechanical stimulus, negative regulation of behavioural response to mechanical stimulus, negative regulation of mechanosensory behaviour, inhibition of behavioral response to mechanical stimulus, inhibition of behavioural response to mechanical stimulus, inhibition of mechanosensory behavior, inhibition of mechanosensory behaviour Definition: Any process that stops, prevents or reduces the frequency, rate or extent of mechanosensory behavior.